Elg1 RFC-like complex [GO:0031391] (cellular component) References: PMID:14614842, PMID:23499004, PMID:27664980 Also known as: Elg1-RFC, Elg1-RLC, RFC (Elg1) Definition: A pentameric replication factor C (RLC) complex, which unloads the DNA polymerase processivity factor proliferating cell nuclear antigen (PCNA) from chromatin and has roles in telomere length regulation and other aspects of genome stability. In Saccharomyces the subunits are known as Elg1p, Rfc2p, Rfc3p, Rfc4p, and Rfc5p. Relationships: is a type of catalytic complex [GO:1902494]; is part of chromosome [GO:0005694]